{
  "term_id": "GO:0006357",
  "term_label": "regulation of transcription by RNA polymerase II",
  "gene_symbol": "SP100",
  "gene_name": "Nuclear autoantigen Sp-100",
  "gene": "UniProtKB:P23497"
}